{
  "gene_symbol": "POU2AF2",
  "term_id": "GO:0005634",
  "term_label": "nucleus",
  "gene": "UniProtKB:Q8IXP5",
  "gene_name": "POU domain class 2-associating factor 2"
}